{
  "gene_name": "Junctional adhesion molecule A",
  "term_label": "bicellular tight junction",
  "term_id": "GO:0005923",
  "gene": "UniProtKB:Q9Y624",
  "gene_symbol": "F11R"
}